maintenance of pole plasm mRNA location [GO:0046594] (biological process) Definition: The process of maintaining mRNA in a specific location in the oocyte pole plasm. An example of this process is found in Drosophila melanogaster. Sources: GOC:bf, GOC:dph, GOC:tb Relationships: is a type of maintenance of RNA location [GO:0051237]; is a type of GO:0051651; BFO_0000050 pole plasm mRNA localization [GO:0019094] Also known as: maintenance of oocyte pole plasm mRNA localization, maintenance of pole plasm mRNA localization